{
  "gene": "UniProtKB:P62263",
  "gene_symbol": "RPS14",
  "term_label": "cytosolic small ribosomal subunit",
  "gene_name": "Small ribosomal subunit protein uS11",
  "term_id": "GO:0022627"
}